(S)-3-amino-2-methylpropionate transaminase activity [GO:0047298] (molecular function) Also known as: (S)-3-amino-2-methylpropionate aminotransferase activity, (S)-3-amino-2-methylpropanoate:2-oxoglutarate aminotransferase activity, L-3-aminoisobutyrate aminotransferase activity, L-3-aminoisobutyrate transaminase activity, L-3-aminoisobutyric aminotransferase activity, L-AIBAT activity, beta-aminobutyric transaminase activity, beta-aminoisobutyrate-alpha-ketoglutarate transaminase activity Definition: Catalysis of the reaction: (S)-3-amino-2-methylpropanoate + 2-oxoglutarate = 2-methyl-3-oxopropanoate + L-glutamate. Relationships: is a type of transaminase activity [GO:0008483] Sources: EC:2.6.1.22, RHEA:13993